{
  "gene": "UniProtKB:Q9BXS0",
  "term_id": "UNKNOWN:0002",
  "term_label": "Unknown biological process",
  "gene_name": "Collagen alpha-1(XXV) chain",
  "gene_symbol": "COL25A1"
}